{
  "term_label": "Golgi apparatus",
  "gene_name": "Polypeptide N-acetylgalactosaminyltransferase 10",
  "gene": "UniProtKB:Q86SR1",
  "gene_symbol": "GALNT10",
  "term_id": "GO:0005794"
}